{
  "term_id": "UNKNOWN:0002",
  "term_label": "Unknown biological process",
  "gene": "UniProtKB:O15488",
  "gene_name": "Glycogenin-2",
  "gene_symbol": "GYG2"
}